plasma membrane raft distribution [GO:0044855] (biological process) Relationships: is a type of GO:0031580; is a type of GO:0044856 Definition: The process that establishes the spatial arrangement of membrane rafts within a plasma membrane. Sources: GOC:jl Subtypes: plasma membrane raft polarization [GO:0044858]